{
  "gene": "UniProtKB:Q8WWY7",
  "gene_name": "WAP four-disulfide core domain protein 12",
  "gene_symbol": "WFDC12",
  "term_id": "GO:0005615",
  "term_label": "extracellular space"
}